callus formation [GO:1990110] (biological process) Definition: The process by which a callus is formed at a wound site. A plant callus is a portion of plant tissue that consists of mass of undifferentiated plant cells. It consists primarily of parenchyma cells but possibly contains other cell types as the callus begins to differentiate. Sources: ISBN:0070187517 Relationships: is a type of multicellular organismal process [GO:0032501]; is part of wound healing [GO:0042060]